aleurone grain [GO:0033095] (cellular component) Relationships: is a type of cytoplasmic vesicle [GO:0031410] References: PMID:22452734 Sources: Wikipedia:Aleurone Definition: A membrane-bounded storage granule found in cells of the aleurone layer in plants; contains either a protein matrix, protein-carbohydrate bodies and/or globoids. Aleurone grains are formed by the vacuole, rough endoplasmic reticulum and dictyosomes. Also known as: aleurone body